positive regulation of F-9775B biosynthetic process [GO:1900677] (biological process) Definition: Any process that activates or increases the frequency, rate or extent of F-9775B biosynthetic process. Sources: GOC:TermGenie, GOC:di Relationships: is a type of regulation of F-9775B biosynthetic process [GO:1900675]; is a type of GO:1900734; positively regulates F-9775B biosynthetic process [GO:1900614] Also known as: activation of F-9775B anabolism, activation of F-9775B biosynthesis, activation of F-9775B formation, activation of F-9775B synthesis, positive regulation of F-9775B anabolism, positive regulation of F-9775B biosynthesis, positive regulation of F-9775B formation, positive regulation of F-9775B synthesis, up regulation of F-9775B anabolism, up regulation of F-9775B biosynthesis, up regulation of F-9775B biosynthetic process, up regulation of F-9775B formation, up regulation of F-9775B synthesis, up-regulation of F-9775B anabolism, up-regulation of F-9775B biosynthesis, up-regulation of F-9775B biosynthetic process, up-regulation of F-9775B formation, up-regulation of F-9775B synthesis, upregulation of F-9775B anabolism, upregulation of F-9775B biosynthesis, upregulation of F-9775B biosynthetic process, upregulation of F-9775B formation, upregulation of F-9775B synthesis, activation of F-9775B biosynthetic process